{
  "gene_name": "Zinc finger protein Aiolos",
  "gene": "UniProtKB:Q9UKT9",
  "term_id": "GO:0000978",
  "term_label": "RNA polymerase II cis-regulatory region sequence-specific DNA binding",
  "gene_symbol": "IKZF3"
}